NAD+ synthase (glutamine-hydrolyzing) activity [GO:0003952] (MF) Relationships: is a type of GO:0016884 Definition: Catalysis of the reaction: deamido-NAD+ + L-glutamine + ATP + H2O = L-glutamate + AMP + diphosphate + NAD+ + H+. Also known as: NAD synthase (glutamine-hydrolyzing) activity, DPN synthetase activity, NAD synthetase (glutamine-hydrolysing), NAD(+) synthetase (glutamine-hydrolyzing) activity, NAD+ synthase (glutamine-hydrolysing), NAD+ synthetase (glutamine-hydrolyzing), deamido-NAD+:L-glutamine amido-ligase (AMP-forming), desamidonicotinamide adenine dinucleotide amidotransferase activity, nicotinamide adenine dinucleotide synthetase (glutamine) activity Sources: RHEA:24384